oxidoreductase activity, acting on other nitrogenous compounds as donors, oxygen as acceptor [GO:0016663] (molecular function) Subtypes: urate oxidase activity [GO:0004846], 3-aci-nitropropanoate oxidase activity [GO:0047557], acetylindoxyl oxidase activity [GO:0047608], hydroxylamine oxidase activity [GO:0047991], GO:0052664 Sources: EC:1.7.3.-, GOC:jl Definition: Catalysis of an oxidation-reduction (redox) reaction in which a nitrogenous group, excluding NH and NH2 groups, acts as a hydrogen or electron donor and reduces oxygen. Relationships: is a type of oxidoreductase activity, acting on other nitrogenous compounds as donors [GO:0016661]